{
  "gene_name": "Leucine-rich alpha-2-glycoprotein",
  "term_label": "type II transforming growth factor beta receptor binding",
  "term_id": "GO:0005114",
  "gene": "UniProtKB:P02750",
  "gene_symbol": "LRG1"
}